{
  "term_id": "GO:0090168",
  "gene_name": "Deubiquitinating protein VCPIP1",
  "term_label": "Golgi reassembly",
  "gene_symbol": "VCPIP1",
  "gene": "UniProtKB:Q96JH7"
}